negative regulation of cardiac muscle cell myoblast differentiation [GO:2000691] (biological process) Relationships: is a type of negative regulation of myoblast differentiation [GO:0045662]; is a type of negative regulation of cardioblast differentiation [GO:0051892]; is a type of regulation of cardiac muscle cell myoblast differentiation [GO:2000690]; RO_0002212 GO:0060379 Also known as: negative regulation of myocardial precursor cell differentiation, negative regulation of cardiac myoblast differentiation Sources: GOC:obol Definition: Any process that stops, prevents or reduces the frequency, rate or extent of cardiac muscle cell myoblast differentiation.